cellular component assembly involved in morphogenesis [GO:0010927] (biological process) Definition: The cellular component assembly that is part of the initial shaping of the component during its developmental progression. Sources: GOC:dph, GOC:tb Relationships: is a type of cellular component assembly [GO:0022607]; is a type of anatomical structure formation involved in morphogenesis [GO:0048646]; is part of cellular anatomical entity morphogenesis [GO:0032989] Subtypes: acrosome assembly [GO:0001675], lamellipodium assembly involved in mesendodermal cell migration [GO:0003364], egg chorion assembly [GO:0007306], pollen wall assembly [GO:0010208], myofibril assembly [GO:0030239], vitelline membrane formation [GO:0030704], paranodal junction assembly [GO:0030913], ascospore-type prospore assembly [GO:0031321], mating projection formation [GO:0031382], GO:0032120, myelin assembly [GO:0032288], cytoneme assembly [GO:0035231], spore wall assembly [GO:0042244], pollen aperture formation [GO:0062075], GO:0071688, mating projection actin fusion focus assembly [GO:1904600], GO:1905499, basement membrane assembly involved in embryonic body morphogenesis [GO:2001197]